{
  "term_label": "Unknown biological process",
  "gene_name": "Mucolipin-1",
  "gene": "UniProtKB:Q9GZU1",
  "term_id": "UNKNOWN:0002",
  "gene_symbol": "MCOLN1"
}